{
  "gene_name": "Keratin-associated protein 6-2",
  "gene_symbol": "KRTAP6-2",
  "term_id": "UNKNOWN:0002",
  "term_label": "Unknown biological process",
  "gene": "UniProtKB:Q3LI66"
}